tetrapyrrole biosynthetic process from glycine and succinyl-CoA [GO:0033527] (biological process) Relationships: is a type of succinyl-CoA metabolic process [GO:0006104]; is a type of glycine metabolic process [GO:0006544]; is a type of tetrapyrrole biosynthetic process [GO:0033014] Regulation: regulated by regulation of tetrapyrrole biosynthetic process from glycine and succinyl-CoA [GO:1901413]; negatively regulated by negative regulation of tetrapyrrole biosynthetic process from glycine and succinyl-CoA [GO:1901414]; positively regulated by positive regulation of tetrapyrrole biosynthetic process from glycine and succinyl-CoA [GO:1901415] Also known as: tetrapyrrole anabolism from glycine and succinyl-CoA, tetrapyrrole biosynthesis from glycine and succinyl-CoA, tetrapyrrole formation from glycine and succinyl-CoA, tetrapyrrole synthesis from glycine and succinyl-CoA Sources: GOC:mah, MetaCyc:PWY-5189 Definition: The chemical reactions and pathways leading to the formation of tetrapyrroles, natural pigments containing four pyrrole rings joined by one-carbon units linking position 2 of one pyrrole ring to position 5 of the next, from other compounds, including glycine and succinyl-CoA.